{
  "term_id": "UNKNOWN:0001",
  "gene_name": "Putative uncharacterized protein ENSP00000383309",
  "term_label": "Unknown molecular function",
  "gene_symbol": "A8MUU9",
  "gene": "UniProtKB:A8MUU9"
}